{
  "gene": "UniProtKB:Q13002",
  "gene_symbol": "GRIK2",
  "term_id": "GO:0015277",
  "gene_name": "Glutamate receptor ionotropic, kainate 2",
  "term_label": "kainate selective glutamate receptor activity"
}